deoxyribonucleoside monophosphate catabolic process [GO:0009159] (biological process) Also known as: deoxyribonucleoside monophosphate breakdown, deoxyribonucleoside monophosphate catabolism, deoxyribonucleoside monophosphate degradation Relationships: is a type of nucleoside monophosphate catabolic process [GO:0009125] Sources: GOC:go_curators, ISBN:0198506732 Definition: The chemical reactions and pathways resulting in the breakdown of a deoxyribonucleoside monophosphate, a compound consisting of a nucleobase linked to a deoxyribose sugar esterified with phosphate on the sugar. Subtypes: purine deoxyribonucleoside monophosphate catabolic process [GO:0009172], pyrimidine deoxyribonucleoside monophosphate catabolic process [GO:0009178]